{
  "gene": "UniProtKB:Q13636",
  "term_label": "GTPase activity",
  "gene_symbol": "RAB31",
  "gene_name": "Ras-related protein Rab-31",
  "term_id": "GO:0003924"
}